{
  "gene": "UniProtKB:Q96T83",
  "gene_name": "Sodium_hydrogen exchanger 7",
  "term_id": "GO:0015385",
  "term_label": "sodium:proton antiporter activity",
  "gene_symbol": "SLC9A7"
}